plasma membrane-derived chromatophore [GO:0042716] (cellular component) Definition: A pigment-bearing structure that is derived from the cytoplasmic membrane, sometimes consisting of simple invaginations and sometimes a complete vesicle. This component is found in certain photosynthetic bacteria and cyanobacteria. References: PMID:11867431 Sources: GOC:jl, ISBN:0395825172 Also known as: chromatophore vesicle Note: Note that this structure is distinct from the chromoplast of plants, which is also sometimes called a chromatophore; it also should not be confused with the specialized pigment-producing cells known as chromatophores, found in fish and amphibian skin. Relationships: is a type of cellular anatomical structure [GO:0110165]; BFO_0000050 cytoplasm [GO:0005737] Subtypes: xanthophore [GO:0031633]